{
  "gene_name": "IQ domain-containing protein E",
  "gene_symbol": "IQCE",
  "term_label": "Unknown cellular component",
  "gene": "UniProtKB:Q6IPM2",
  "term_id": "UNKNOWN:0003"
}